{
  "term_label": "Unknown molecular function",
  "gene": "UniProtKB:Q7Z6K5",
  "gene_name": "Arpin",
  "term_id": "UNKNOWN:0001",
  "gene_symbol": "ARPIN"
}